{
  "gene_symbol": "HOMER1",
  "gene_name": "Homer protein homolog 1",
  "term_label": "G protein-coupled glutamate receptor binding",
  "gene": "UniProtKB:Q86YM7",
  "term_id": "GO:0035256"
}